{
  "gene_symbol": "RILPL2",
  "gene_name": "RILP-like protein 2",
  "term_label": "cytoplasm",
  "term_id": "GO:0005737",
  "gene": "UniProtKB:Q969X0"
}